heteroduplex formation [GO:0030491] (biological process) Relationships: is_a GO:0006259 Subtypes: heteroduplex formation involved in double-strand break repair via synthesis-dependent strand annealing [GO:0010709] References: PMID:10357855 Sources: GOC:elh Definition: The formation of a stable duplex DNA that contains one strand from each of the two recombining DNA molecules.